{
  "gene_symbol": "PRAMEF1",
  "term_label": "Cul2-RING ubiquitin ligase complex",
  "gene_name": "PRAME family member 1",
  "term_id": "GO:0031462",
  "gene": "UniProtKB:O95521"
}